{
  "term_id": "GO:0005787",
  "term_label": "signal peptidase complex",
  "gene_name": "Signal peptidase complex subunit 2",
  "gene_symbol": "SPCS2",
  "gene": "UniProtKB:Q15005"
}